{
  "term_id": "GO:0000976",
  "gene_name": "Zinc finger protein 729",
  "gene": "UniProtKB:A6NN14",
  "term_label": "transcription cis-regulatory region binding",
  "gene_symbol": "ZNF729"
}